asymmetric protein localization involved in cell fate determination [GO:0045167] (biological process) Relationships: is_a intracellular protein localization [GO:0008104]; is part of GO:0001709 Regulation: regulated by regulation of asymmetric protein localization involved in cell fate determination [GO:1904785]; RO_0002212 by negative regulation of asymmetric protein localization involved in cell fate determination [GO:1904786]; positively regulated by positive regulation of asymmetric protein localization involved in cell fate determination [GO:1904787] Definition: Any process in which a protein is transported to, or maintained in, a specific asymmetric distribution, resulting in the formation of daughter cells of different types. Also known as: asymmetric protein localisation involved in cell fate determination, asymmetric protein localization involved in cell fate commitment, asymmetric protein localization resulting in cell fate commitment, cell fate commitment, asymmetric protein localization Sources: GOC:ai